{
  "gene": "UniProtKB:Q8NE86",
  "term_label": "calcium import into the mitochondrion",
  "term_id": "GO:0036444",
  "gene_name": "Calcium uniporter protein, mitochondrial",
  "gene_symbol": "MCU"
}